{
  "gene": "UniProtKB:Q8IWT1",
  "gene_name": "Sodium channel subunit beta-4",
  "term_label": "cardiac muscle cell action potential involved in contraction",
  "gene_symbol": "SCN4B",
  "term_id": "GO:0086002"
}